{
  "gene": "UniProtKB:Q9NQQ7",
  "term_id": "GO:0005801",
  "gene_name": "Solute carrier family 35 member C2",
  "term_label": "cis-Golgi network",
  "gene_symbol": "SLC35C2"
}